{
  "gene_name": "Uncharacterized protein KIAA1143",
  "term_id": "UNKNOWN:0003",
  "gene_symbol": "KIAA1143",
  "term_label": "Unknown cellular component",
  "gene": "UniProtKB:Q96AT1"
}